{
  "term_id": "UNKNOWN:0001",
  "term_label": "Unknown molecular function",
  "gene": "UniProtKB:Q9UDX4",
  "gene_symbol": "SEC14L3",
  "gene_name": "SEC14-like protein 3"
}